{
  "gene": "UniProtKB:Q8WV24",
  "gene_name": "Pleckstrin homology-like domain family A member 1",
  "gene_symbol": "PHLDA1",
  "term_label": "positive regulation of apoptotic process",
  "term_id": "GO:0043065"
}